serotonin metabolic process [GO:0042428] (biological process) Definition: The chemical reactions and pathways involving serotonin (5-hydroxytryptamine), a monoamine neurotransmitter occurring in the peripheral and central nervous systems, also having hormonal properties. Sources: GOC:jl, ISBN:0198506732 Relationships: is a type of phenol-containing compound metabolic process [GO:0018958]; is a type of indole-containing compound metabolic process [GO:0042430] Subtypes: GO:0042427, serotonin catabolic process [GO:0042429] Also known as: serotonin metabolism